{
  "gene_symbol": "PDGFB",
  "gene_name": "Platelet-derived growth factor subunit B",
  "term_label": "extracellular space",
  "gene": "UniProtKB:P01127",
  "term_id": "GO:0005615"
}